{
  "gene_name": "Citramalyl-CoA lyase, mitochondrial",
  "gene": "UniProtKB:Q8N0X4",
  "term_id": "GO:0106064",
  "term_label": "regulation of cobalamin metabolic process",
  "gene_symbol": "CLYBL"
}